{
  "gene_symbol": "LGALS3",
  "gene_name": "Galectin-3",
  "gene": "UniProtKB:P17931",
  "term_id": "GO:2001237",
  "term_label": "negative regulation of extrinsic apoptotic signaling pathway"
}